{
  "gene_symbol": "CT45A9",
  "term_label": "Unknown molecular function",
  "gene": "UniProtKB:P0DMV2",
  "term_id": "UNKNOWN:0001",
  "gene_name": "Cancer_testis antigen family 45 member A9"
}